{
  "term_label": "synaptic vesicle fusion to presynaptic active zone membrane",
  "term_id": "GO:0031629",
  "gene_symbol": "SNAP23",
  "gene": "UniProtKB:O00161",
  "gene_name": "Synaptosomal-associated protein 23"
}